{
  "term_id": "UNKNOWN:0001",
  "term_label": "Unknown molecular function",
  "gene_name": "Putative uncharacterized protein FLJ46204",
  "gene_symbol": "Q6ZRP5",
  "gene": "UniProtKB:Q6ZRP5"
}